{
  "term_label": "innate immune response in mucosa",
  "gene_symbol": "DEFB1",
  "term_id": "GO:0002227",
  "gene_name": "Beta-defensin 1",
  "gene": "UniProtKB:P60022"
}